{
  "term_id": "GO:0005615",
  "term_label": "extracellular space",
  "gene_symbol": "UMOD",
  "gene_name": "Uromodulin",
  "gene": "UniProtKB:P07911"
}